maleylpyruvate hydrolase activity [GO:0102054] (MF) Definition: Catalysis of the reaction: 3-maleylpyruvate(2-) + H2O = H+ + maleate(2-) + pyruvate. References: PMID:7400101 Sources: GOC:pz, RHEA:47956 Relationships: is a type of GO:0016823